negative regulation of pancreatic amylase secretion [GO:1902277] (biological process) Also known as: down regulation of pancreatic amylase secretion, down-regulation of pancreatic amylase secretion, downregulation of pancreatic amylase secretion, inhibition of pancreatic amylase secretion Definition: Any process that stops, prevents or reduces the frequency, rate or extent of pancreatic amylase secretion. Sources: GOC:TermGenie, GOC:jc Relationships: is_a negative regulation of protein secretion [GO:0050709]; is a type of GO:1902276; negatively regulates GO:0036395